{
  "term_label": "RQC-trigger complex",
  "gene": "UniProtKB:Q15650",
  "gene_symbol": "TRIP4",
  "gene_name": "Activating signal cointegrator 1",
  "term_id": "GO:0180022"
}